{
  "term_id": "GO:0031462",
  "gene": "UniProtKB:Q5VTA0",
  "term_label": "Cul2-RING ubiquitin ligase complex",
  "gene_symbol": "PRAMEF17",
  "gene_name": "PRAME family member 17"
}